{
  "term_id": "GO:0043122",
  "gene_symbol": "TRAF4",
  "term_label": "regulation of canonical NF-kappaB signal transduction",
  "gene": "UniProtKB:Q9BUZ4",
  "gene_name": "TNF receptor-associated factor 4"
}